negative regulation of calcium-independent cell-cell adhesion [GO:0051042] (biological process) Also known as: down regulation of calcium-independent cell-cell adhesion, down-regulation of calcium-independent cell-cell adhesion, downregulation of calcium-independent cell-cell adhesion, inhibition of calcium-independent cell-cell adhesion Sources: GOC:ai Relationships: is a type of negative regulation of cell-cell adhesion [GO:0022408]; is a type of GO:0051040; negatively regulates calcium-independent cell-cell adhesion [GO:0016338] Definition: Any process that stops, prevents, or reduces the frequency, rate or extent of calcium-independent cell-cell adhesion.